{
  "term_id": "UNKNOWN:0003",
  "gene_symbol": "F13A1",
  "gene": "UniProtKB:P00488",
  "term_label": "Unknown cellular component",
  "gene_name": "Coagulation factor XIII A chain"
}